{
  "gene_name": "Protein myomixer",
  "gene": "UniProtKB:A0A1B0GTQ4",
  "term_label": "Golgi membrane",
  "term_id": "GO:0000139",
  "gene_symbol": "MYMX"
}